{
  "gene": "UniProtKB:P55060",
  "gene_symbol": "CSE1L",
  "term_id": "GO:0005829",
  "term_label": "cytosol",
  "gene_name": "Exportin-2"
}